{
  "term_id": "GO:0005730",
  "gene_name": "Protein RRP5 homolog",
  "term_label": "nucleolus",
  "gene_symbol": "PDCD11",
  "gene": "UniProtKB:Q14690"
}